{
  "term_label": "plasma membrane",
  "gene_symbol": "RAB8A",
  "term_id": "GO:0005886",
  "gene": "UniProtKB:P61006",
  "gene_name": "Ras-related protein Rab-8A"
}